{
  "term_id": "UNKNOWN:0003",
  "term_label": "Unknown cellular component",
  "gene": "UniProtKB:Q5JQS6",
  "gene_symbol": "GCSAML",
  "gene_name": "Germinal center-associated signaling and motility-like protein"
}